UTP metabolic process [GO:0046051] (BP) Also known as: UTP metabolism Subtypes: UTP biosynthetic process [GO:0006228], GO:0046052 Relationships: is a type of GO:0009208; is a type of pyrimidine ribonucleotide metabolic process [GO:0009218] Sources: GOC:go_curators Definition: The chemical reactions and pathways involving UTP, uridine (5'-)triphosphate.